{
  "gene": "UniProtKB:Q9Y6I3",
  "term_id": "GO:0005886",
  "gene_symbol": "EPN1",
  "gene_name": "Epsin-1",
  "term_label": "plasma membrane"
}